{
  "gene": "UniProtKB:Q06787",
  "term_id": "GO:0048513",
  "term_label": "animal organ development",
  "gene_name": "Fragile X messenger ribonucleoprotein 1",
  "gene_symbol": "FMR1"
}